{
  "gene_symbol": "MRPL21",
  "term_label": "Unknown biological process",
  "gene_name": "Large ribosomal subunit protein bL21m",
  "term_id": "UNKNOWN:0002",
  "gene": "UniProtKB:Q7Z2W9"
}